phosphoacetylglucosamine mutase activity [GO:0004610] (MF) Also known as: N-acetyl-D-glucosamine 1,6-phosphomutase activity, N-acetyl-alpha-D-glucosamine 1,6-phosphomutase activity, N-acetylglucosamine-phosphate mutase activity, acetylaminodeoxyglucose phosphomutase activity, acetylglucosamine phosphomutase activity, phospho-N-acetylglucosamine mutase activity Definition: Catalysis of the reaction: N-acetyl-alpha-D-glucosamine 1-phosphate = N-acetyl-D-glucosamine 6-phosphate. Relationships: is a type of intramolecular phosphotransferase activity [GO:0016868] Sources: EC:5.4.2.3, RHEA:23804